{
  "gene_symbol": "USP17L5",
  "gene_name": "Ubiquitin carboxyl-terminal hydrolase 17-like protein 5",
  "term_id": "GO:0031647",
  "gene": "UniProtKB:A8MUK1",
  "term_label": "regulation of protein stability"
}